DNA integration [GO:0015074] (biological process) Sources: GOC:mah Relationships: is a type of DNA metabolic process [GO:0006259] Definition: The process in which a DNA segment is incorporated into another, usually larger, DNA molecule such as a chromosome.